{
  "gene_symbol": "KIR2DL1",
  "gene": "UniProtKB:A0A191URJ7",
  "term_id": "GO:0005886",
  "term_label": "plasma membrane",
  "gene_name": "KIR2DL protein"
}